{
  "term_label": "regulation of actin filament polymerization",
  "gene_symbol": "FCHSD1",
  "gene": "UniProtKB:Q86WN1",
  "gene_name": "F-BAR and double SH3 domains protein 1",
  "term_id": "GO:0030833"
}